{
  "term_label": "positive regulation of insulin secretion involved in cellular response to glucose stimulus",
  "gene": "UniProtKB:O14523",
  "gene_name": "Phospholipid transfer protein C2CD2L",
  "gene_symbol": "C2CD2L",
  "term_id": "GO:0035774"
}